myo-inositol import across plasma membrane [GO:1904679] (biological process) Definition: The directed movement of myo-inositol from outside of a cell, across the plasma membrane and into the cytosol. References: PMID:9560432 Sources: GOC:TermGenie, GO_REF:0000075 Also known as: myo-inositol import into cell Relationships: is a type of GO:0015791; is a type of myo-inositol transport [GO:0015798]; is a type of GO:0098739